{
  "term_id": "GO:0006493",
  "gene_name": "Protein O-mannose kinase",
  "gene": "UniProtKB:Q9H5K3",
  "gene_symbol": "POMK",
  "term_label": "protein O-linked glycosylation"
}